negative regulation of protein import into nucleus [GO:0042308] (biological process) Sources: GOC:jl Definition: Any process that stops, prevents, or reduces the frequency, rate or extent of the movement of proteins from the cytoplasm into the nucleus. Relationships: is a type of GO:0042306; is a type of negative regulation of nucleocytoplasmic transport [GO:0046823]; is a type of negative regulation of intracellular protein transport [GO:0090317]; is a type of GO:1900181; negatively regulates protein import into nucleus [GO:0006606] Also known as: down regulation of protein import into nucleus, down-regulation of protein import into nucleus, downregulation of protein import into nucleus, negative regulation of protein import into cell nucleus, negative regulation of protein transport from cytoplasm to nucleus, negative regulation of protein-nucleus import, inhibition of protein import into nucleus